phagocytic cup lip [GO:0097203] (cellular component) References: PMID:20200225 Sources: GOC:pf Definition: The tip or margin of the progressing circular lamella that engulfs a particle during phagocytosis. When the two lips of the cup fuse it is converted into a phagosome. Relationships: is a type of GO:0110165; is part of phagocytic cup [GO:0001891]